{
  "term_label": "translation release factor complex",
  "gene_symbol": "GSPT1",
  "term_id": "GO:0018444",
  "gene_name": "Eukaryotic peptide chain release factor GTP-binding subunit ERF3A",
  "gene": "UniProtKB:P15170"
}